virus tail fiber assembly [GO:0098004] (biological process) Relationships: is a type of viral process [GO:0016032]; is part of viral tail assembly [GO:0098003] Definition: The aggregation, arrangement and bonding together of a set of components to form a virus tail fiber. Sources: GOC:bm, VZ:3956